{
  "gene_name": "Large ribosomal subunit protein uL13m",
  "gene_symbol": "MRPL13",
  "term_label": "negative regulation of translation",
  "term_id": "GO:0017148",
  "gene": "UniProtKB:Q9BYD1"
}